{
  "gene_name": "Spindlin-4",
  "gene": "UniProtKB:Q56A73",
  "term_label": "regulation of DNA-templated transcription",
  "term_id": "GO:0006355",
  "gene_symbol": "SPIN4"
}